{
  "term_label": "regulation of mitochondrial mRNA stability",
  "gene_name": "FAST kinase domain-containing protein 2, mitochondrial",
  "term_id": "GO:0044528",
  "gene": "UniProtKB:Q9NYY8",
  "gene_symbol": "FASTKD2"
}